{
  "gene": "UniProtKB:O60524",
  "term_label": "ribosomal large subunit binding",
  "term_id": "GO:0043023",
  "gene_name": "Ribosome quality control complex subunit NEMF",
  "gene_symbol": "NEMF"
}